{
  "gene": "UniProtKB:A1L170",
  "gene_name": "Uncharacterized protein C1orf226",
  "gene_symbol": "C1orf226",
  "term_label": "Unknown molecular function",
  "term_id": "UNKNOWN:0001"
}